{
  "term_id": "UNKNOWN:0002",
  "gene": "UniProtKB:Q5T6X5",
  "gene_symbol": "GPRC6A",
  "gene_name": "G-protein coupled receptor family C group 6 member A",
  "term_label": "Unknown biological process"
}